{
  "gene": "UniProtKB:P16278",
  "gene_name": "Beta-galactosidase",
  "gene_symbol": "GLB1",
  "term_label": "vacuole",
  "term_id": "GO:0005773"
}